extraction of mislocalized protein from membrane [GO:0140568] (biological process) Relationships: is a type of establishment of protein localization to membrane [GO:0090150] Definition: The removal of a mislocalized protein from a cellular membrane. Subtypes: extraction of mislocalized protein from ER membrane [GO:0140569], extraction of mislocalized protein from mitochondrial outer membrane [GO:0140570] References: PMID:24821790, PMID:28712723, PMID:32973005